{
  "term_id": "GO:0000976",
  "gene_symbol": "ZNF226",
  "gene": "UniProtKB:Q9NYT6",
  "gene_name": "Zinc finger protein 226",
  "term_label": "transcription cis-regulatory region binding"
}